{
  "term_id": "GO:0005743",
  "gene_name": "Solute carrier family 25 member 3",
  "term_label": "mitochondrial inner membrane",
  "gene": "UniProtKB:Q00325",
  "gene_symbol": "SLC25A3"
}